superior endocardial cushion morphogenesis [GO:1905316] (biological process) Definition: The developmental process by which a superior endocardial cushion is generated and organized. Also known as: dorsal endocardial cushion morphogenesis Relationships: is a type of endocardial cushion morphogenesis [GO:0003203] References: PMID:17050629 Sources: GOC:BHF, GOC:TermGenie, GOC:rl, GO_REF:0000083